{
  "gene_name": "Calcium release-activated calcium channel protein 1",
  "term_label": "store-operated calcium entry",
  "gene": "UniProtKB:Q96D31",
  "gene_symbol": "ORAI1",
  "term_id": "GO:0002115"
}